{
  "term_label": "Unknown molecular function",
  "term_id": "UNKNOWN:0001",
  "gene": "UniProtKB:Q6UWM5",
  "gene_symbol": "GLIPR1L1",
  "gene_name": "GLIPR1-like protein 1"
}